replacement bone morphogenesis [GO:0061971] (biological process) Relationships: is a type of bone morphogenesis [GO:0060349] References: PMID:29852585 Definition: The process in which bones are generated and organized as a result of the conversion of another structural tissue into bone.